{
  "gene_symbol": "PITPNM1",
  "gene": "UniProtKB:O00562",
  "gene_name": "Membrane-associated phosphatidylinositol transfer protein 1",
  "term_label": "Unknown biological process",
  "term_id": "UNKNOWN:0002"
}